{
  "gene_symbol": "OR11H12",
  "term_label": "Unknown biological process",
  "term_id": "UNKNOWN:0002",
  "gene_name": "Olfactory receptor 11H12",
  "gene": "UniProtKB:B2RN74"
}